{
  "term_id": "UNKNOWN:0003",
  "gene_name": "Zinc finger Ran-binding domain-containing protein 2",
  "gene_symbol": "ZRANB2",
  "gene": "UniProtKB:O95218",
  "term_label": "Unknown cellular component"
}